{
  "gene_name": "Collagen alpha-1(XV) chain",
  "gene_symbol": "COL15A1",
  "gene": "UniProtKB:P39059",
  "term_label": "extracellular matrix organization",
  "term_id": "GO:0030198"
}